{
  "gene_symbol": "VPS4B",
  "gene_name": "Vacuolar protein sorting-associated protein 4B",
  "gene": "UniProtKB:O75351",
  "term_id": "GO:0005737",
  "term_label": "cytoplasm"
}